{
  "gene_symbol": "RASSF2",
  "gene": "UniProtKB:P50749",
  "term_id": "GO:0005737",
  "gene_name": "Ras association domain-containing protein 2",
  "term_label": "cytoplasm"
}